pyridoxal phosphate transmembrane transporter activity [GO:0031926] (molecular function) Definition: Enables the transfer of pyridoxal phosphate from one side of a membrane to the other. Pyridoxal phosphate is pyridoxal phosphorylated at the hydroxymethyl group of C-5, and is the active form of vitamin B6. Relationships: is a type of organophosphate ester transmembrane transporter activity [GO:0015605] Sources: GOC:mah